{
  "term_id": "GO:0018685",
  "gene_name": "Cytochrome P450 4A11",
  "gene_symbol": "CYP4A11",
  "gene": "UniProtKB:Q02928",
  "term_label": "alkane 1-monooxygenase activity"
}